{
  "gene_symbol": "OR8H2",
  "gene_name": "Olfactory receptor 8H2",
  "term_id": "GO:0007186",
  "gene": "UniProtKB:Q8N162",
  "term_label": "G protein-coupled receptor signaling pathway"
}